{
  "gene": "UniProtKB:Q969R8",
  "gene_symbol": "ITFG2",
  "term_label": "regulation of TOR signaling",
  "term_id": "GO:0032006",
  "gene_name": "KICSTOR complex protein ITFG2"
}